{
  "gene": "UniProtKB:Q6Q4G3",
  "term_label": "metalloaminopeptidase activity",
  "term_id": "GO:0070006",
  "gene_symbol": "LVRN",
  "gene_name": "Aminopeptidase Q"
}